{
  "gene": "UniProtKB:Q92771",
  "term_label": "establishment of sister chromatid cohesion",
  "term_id": "GO:0034085",
  "gene_name": "Putative ATP-dependent RNA helicase DDX12",
  "gene_symbol": "DDX12P"
}